{
  "gene_name": "Inactive N-acetyllactosaminide alpha-1,3-galactosyltransferase",
  "gene": "UniProtKB:Q4G0N0",
  "term_id": "UNKNOWN:0003",
  "term_label": "Unknown cellular component",
  "gene_symbol": "GGTA1"
}